regulation of plant epidermal cell differentiation [GO:1903888] (BP) References: PMID:123345 Sources: GOC:TermGenie, GO_REF:0000058 Relationships: is a type of regulation of cell differentiation [GO:0045595]; RO_0002211 plant epidermal cell differentiation [GO:0090627] Subtypes: regulation of atrichoblast fate specification [GO:0010058], regulation of trichoblast fate specification [GO:0010061], negative regulation of plant epidermal cell differentiation [GO:1903889], positive regulation of plant epidermal cell differentiation [GO:1903890] Definition: Any process that modulates the frequency, rate or extent of plant epidermal cell differentiation.